{
  "gene": "UniProtKB:Q5SSQ6",
  "gene_symbol": "SAPCD1",
  "term_label": "Unknown biological process",
  "term_id": "UNKNOWN:0002",
  "gene_name": "Suppressor APC domain-containing protein 1"
}